{
  "term_label": "septin ring",
  "gene_name": "Septin-9",
  "term_id": "GO:0005940",
  "gene_symbol": "SEPTIN9",
  "gene": "UniProtKB:Q9UHD8"
}